cellular response to virus [GO:0098586] (biological process) Sources: GOC:dos Definition: Any process that results in a change in state or activity of a cell (in terms of movement, secretion, enzyme production, gene expression, etc.) as a result of a stimulus from a virus. Relationships: is_a response to virus [GO:0009615]